{
  "gene": "UniProtKB:O75787",
  "term_id": "GO:0030177",
  "gene_symbol": "ATP6AP2",
  "term_label": "positive regulation of Wnt signaling pathway",
  "gene_name": "Renin receptor"
}